{
  "gene_symbol": "NIN",
  "gene": "UniProtKB:Q8N4C6",
  "term_label": "centrosome-templated microtubule nucleation",
  "term_id": "GO:0090222",
  "gene_name": "Ninein"
}